{
  "term_label": "adherens junction",
  "term_id": "GO:0005912",
  "gene_symbol": "NECTIN4",
  "gene": "UniProtKB:Q96NY8",
  "gene_name": "Nectin-4"
}